{
  "gene_symbol": "HBA2",
  "gene": "UniProtKB:P69905",
  "term_id": "GO:0015671",
  "term_label": "oxygen transport",
  "gene_name": "Hemoglobin subunit alpha"
}